{
  "term_id": "GO:0008210",
  "gene_symbol": "UGT2B28",
  "gene_name": "UDP-glucuronosyltransferase 2B28",
  "term_label": "estrogen metabolic process",
  "gene": "UniProtKB:Q9BY64"
}